{
  "gene": "UniProtKB:Q96CC6",
  "term_id": "GO:0050708",
  "gene_symbol": "RHBDF1",
  "term_label": "regulation of protein secretion",
  "gene_name": "Inactive rhomboid protein 1"
}